{
  "gene_name": "Cyclin-J",
  "term_label": "G1/S transition of mitotic cell cycle",
  "gene_symbol": "CCNJ",
  "term_id": "GO:0000082",
  "gene": "UniProtKB:Q5T5M9"
}